symbiont entry into host cell via disruption of host cell envelope lipopolysaccharide [GO:0098995] (biological process) Sources: GOC:dos, VZ:3940 Relationships: is a type of symbiont-mediated disruption of host cell wall [GO:0052009]; is part of symbiont entry into host cell [GO:0046718] Definition: The disruption by a symbiont of host cell wall lipopolysaccharides to allow entry into the host cell. For example a phage entering a Gram-negative bacterium may actively break down outer membrane lipopolysaccharides. Also known as: degradation of host cell envelope lipopolysaccharide during viral entry, degradation of host lipopolysaccharide during virus entry, disruption by virus of host envelope lipopolysaccharide during virus entry, disassembly by virus of outer membrane lipopolysaccharide during viral entry